{
  "term_id": "GO:0005737",
  "term_label": "cytoplasm",
  "gene": "UniProtKB:Q14449",
  "gene_name": "Growth factor receptor-bound protein 14",
  "gene_symbol": "GRB14"
}